nucleobase-containing small molecule catabolic process [GO:0034656] (biological process) Also known as: nucleobase, nucleoside and nucleotide breakdown, nucleobase, nucleoside and nucleotide catabolism, nucleobase, nucleoside and nucleotide degradation Sources: GOC:mah Relationships: is a type of nucleobase-containing compound catabolic process [GO:0034655]; is a type of GO:0044282; is a type of nucleobase-containing small molecule metabolic process [GO:0055086] Definition: The chemical reactions and pathways resulting in the breakdown of a nucleobase-containing small molecule: a nucleobase, a nucleoside, or a nucleotide. Subtypes: nucleoside catabolic process [GO:0009164]